negative regulation of insulin secretion [GO:0046676] (biological process) Sources: GOC:ai Definition: Any process that stops, prevents, or reduces the frequency, rate or extent of the regulated release of insulin. Also known as: down regulation of insulin secretion, down-regulation of insulin secretion, downregulation of insulin secretion, inhibition of insulin secretion Subtypes: GO:0061179 Relationships: is a type of negative regulation of protein secretion [GO:0050709]; is_a regulation of insulin secretion [GO:0050796]; is a type of negative regulation of peptide hormone secretion [GO:0090278]; negatively regulates insulin secretion [GO:0030073]